{
  "term_label": "prostaglandin D receptor activity",
  "gene": "UniProtKB:Q9Y5Y4",
  "term_id": "GO:0004956",
  "gene_symbol": "PTGDR2",
  "gene_name": "Prostaglandin D2 receptor 2"
}